negative regulation of potassium ion transport [GO:0043267] (biological process) Relationships: is a type of GO:0043266; is a type of negative regulation of monoatomic ion transport [GO:0043271]; negatively regulates GO:0006813 Subtypes: negative regulation of potassium ion transmembrane transport [GO:1901380] Definition: Any process that stops, prevents, or reduces the frequency, rate or extent of the directed movement of potassium ions (K+) into, out of or within a cell, or between cells, by means of some agent such as a transporter or pore. Also known as: down regulation of potassium ion transport, down-regulation of potassium ion transport, downregulation of potassium ion transport, negative regulation of K+ transport, negative regulation of potassium transport, inhibition of potassium ion transport, negative regulation of potassium ion conductance, regulation of K+ conductance, regulation of potassium conductance, transmembrane conductance regulator activity Sources: GOC:jl